negative regulation of cholesterol import [GO:0060621] (biological process) Definition: Any process that decreases the rate, frequency or extent of cholesterol import. Cholesterol import is the directed movement of cholesterol into a cell or organelle. Relationships: is a type of negative regulation of cholesterol transport [GO:0032375]; is a type of regulation of cholesterol import [GO:0060620]; negatively regulates cholesterol import [GO:0070508] Sources: GOC:BHF, GOC:dph, GOC:tb